adenylate cyclase-inhibiting G protein-coupled acetylcholine receptor signaling pathway [GO:0007197] (biological process) Sources: GOC:dph, GOC:mah, GOC:signaling, GOC:tb Relationships: is a type of adenylate cyclase-inhibiting G protein-coupled receptor signaling pathway [GO:0007193]; is a type of GO:0007213 Definition: An adenylate cyclase-inhibiting G protein-coupled receptor signaling pathway initiated by acetylcholine binding to its receptor, and ending with the regulation of a downstream cellular process. Also known as: muscarinic acetylcholine receptor, adenylate cyclase inhibiting pathway, muscarinic acetylcholine receptor, adenylyl cyclase inhibiting pathway, inhibition of adenylate cyclase activity by G-protein coupled acetylcholine receptor signaling pathway, inhibition of adenylate cyclase activity by muscarinic acetylcholine receptor signaling pathway, inhibition of adenylate cyclase activity by muscarinic acetylcholine receptor signalling pathway